{
  "gene": "UniProtKB:Q9NQZ7",
  "gene_name": "Ectonucleoside triphosphate diphosphohydrolase 7",
  "term_label": "membrane",
  "gene_symbol": "ENTPD7",
  "term_id": "GO:0016020"
}